{
  "term_label": "basolateral plasma membrane",
  "gene_symbol": "SLC4A11",
  "gene_name": "Solute carrier family 4 member 11",
  "gene": "UniProtKB:Q8NBS3",
  "term_id": "GO:0016323"
}